negative regulation of intrinsic apoptotic signaling pathway in response to osmotic stress by p53 class mediator [GO:1902239] (biological process) Relationships: is a type of negative regulation of intrinsic apoptotic signaling pathway in response to osmotic stress [GO:1902219]; is a type of GO:1902238; is a type of GO:1902254; negatively regulates intrinsic apoptotic signaling pathway in response to osmotic stress by p53 class mediator [GO:1990127] Also known as: down regulation of intrinsic apoptotic signaling pathway in response to osmotic stress by p53 class mediator, down-regulation of intrinsic apoptotic signaling pathway in response to osmotic stress by p53 class mediator, downregulation of intrinsic apoptotic signaling pathway in response to osmotic stress by p53 class mediator, inhibition of intrinsic apoptotic signaling pathway in response to osmotic stress by p53 class mediator Definition: Any process that stops, prevents or reduces the frequency, rate or extent of intrinsic apoptotic signaling pathway in response to osmotic stress by p53 class mediator. References: PMID:16571598 Sources: GOC:TermGenie, GOC:krc, GOC:mtg_apoptosis